{
  "gene_symbol": "PCDH18",
  "gene_name": "Protocadherin-18",
  "term_label": "cell adhesion molecule binding",
  "term_id": "GO:0050839",
  "gene": "UniProtKB:Q9HCL0"
}